{
  "gene_symbol": "PP632",
  "term_id": "UNKNOWN:0002",
  "term_label": "Unknown biological process",
  "gene": "UniProtKB:Q6XCG6",
  "gene_name": "Putative uncharacterized protein PP632"
}